{
  "gene": "UniProtKB:Q15393",
  "gene_symbol": "SF3B3",
  "gene_name": "Splicing factor 3B subunit 3",
  "term_label": "nucleus",
  "term_id": "GO:0005634"
}